{
  "gene_symbol": "PROC",
  "gene": "UniProtKB:P04070",
  "term_label": "extracellular space",
  "gene_name": "Vitamin K-dependent protein C",
  "term_id": "GO:0005615"
}